{
  "gene": "UniProtKB:Q6XPR3",
  "gene_name": "Repetin",
  "gene_symbol": "RPTN",
  "term_id": "UNKNOWN:0001",
  "term_label": "Unknown molecular function"
}